{
  "term_label": "Unknown cellular component",
  "gene_name": "T-cell leukemia_lymphoma protein 1B",
  "gene": "UniProtKB:O95988",
  "term_id": "UNKNOWN:0003",
  "gene_symbol": "TCL1B"
}